{
  "gene_name": "E3 ubiquitin-protein ligase RNF139",
  "term_label": "Derlin-1 retrotranslocation complex",
  "gene": "UniProtKB:Q8WU17",
  "gene_symbol": "RNF139",
  "term_id": "GO:0036513"
}